beta-diketone hydrolase activity [GO:0047699] (molecular function) Also known as: b-diketone hydrolase activity, nonane-4,6-dione acylhydrolase activity, oxidized PVA hydrolase activity Relationships: is a type of hydrolase activity, acting on acid carbon-carbon bonds, in ketonic substances [GO:0016823] Definition: Catalysis of the reaction: H2O + nonane-4,6-dione = butanoate + H+ + pentan-2-one. Sources: RHEA:11908